negative regulation of glucagon secretion [GO:0070093] (biological process) Sources: GOC:BHF, GOC:mah Also known as: down regulation of glucagon secretion, down-regulation of glucagon secretion, downregulation of glucagon secretion, inhibition of glucagon secretion Relationships: is a type of regulation of glucagon secretion [GO:0070092]; is a type of GO:0090278; negatively regulates GO:0070091 Definition: Any process that stops, prevents, or reduces the frequency, rate or extent of the regulated release of glucagon.